{
  "term_label": "plasma membrane",
  "gene_name": "Solute carrier family 52, riboflavin transporter, member 1",
  "gene": "UniProtKB:Q9NWF4",
  "term_id": "GO:0005886",
  "gene_symbol": "SLC52A1"
}